{
  "gene_symbol": "EPPK1",
  "gene": "UniProtKB:P58107",
  "term_id": "GO:0016020",
  "term_label": "membrane",
  "gene_name": "Epiplakin"
}